{
  "term_label": "proteasome-mediated ubiquitin-dependent protein catabolic process",
  "gene_symbol": "SPSB4",
  "term_id": "GO:0043161",
  "gene": "UniProtKB:Q96A44",
  "gene_name": "SPRY domain-containing SOCS box protein 4"
}